{
  "term_label": "negative regulation of endothelial cell proliferation",
  "gene_name": "Caveolin-2",
  "gene": "UniProtKB:P51636",
  "gene_symbol": "CAV2",
  "term_id": "GO:0001937"
}